{
  "term_id": "GO:0007157",
  "gene_symbol": "SELP",
  "gene_name": "P-selectin",
  "term_label": "heterophilic cell-cell adhesion",
  "gene": "UniProtKB:P16109"
}